response to continuous far red light stimulus by the high-irradiance response system [GO:0010201] (biological process) Relationships: is a type of response to far red light [GO:0010218] Definition: Any process that results in a change in state or activity of a cell or an organism (in terms of movement, secretion, enzyme production, gene expression, etc.) as a result of the detection of a continuous far red light stimulus by the high-irradiance response system. Far red light is electromagnetic radiation of wavelength 700-800nm. The activity of the high-irradiance response system is characterized by stronger effects of continuous than pulsed light at equal total fluence. Sources: GOC:mtg_far_red, GOC:sm